{
  "gene": "UniProtKB:Q86UT6",
  "term_id": "GO:0043124",
  "gene_name": "NLR family member X1",
  "term_label": "negative regulation of canonical NF-kappaB signal transduction",
  "gene_symbol": "NLRX1"
}